{
  "gene_symbol": "BHMT2",
  "term_id": "GO:0005829",
  "term_label": "cytosol",
  "gene": "UniProtKB:Q9H2M3",
  "gene_name": "S-methylmethionine--homocysteine S-methyltransferase BHMT2"
}